respiratory system process [GO:0003016] (biological process) Subtypes: GO:0002086, mucociliary clearance [GO:0120197] Relationships: is a type of GO:0003008; is part of respiratory gaseous exchange by respiratory system [GO:0007585] Also known as: respiratory gaseous exchange Sources: GOC:dph, GOC:mtg_cardio, GOC:tb Definition: A process carried out by the organs or tissues of the respiratory system. The respiratory system is an organ system responsible for respiratory gaseous exchange. Regulation: regulated by regulation of respiratory system process [GO:0044065]